{
  "term_label": "regulation of transcription by RNA polymerase II",
  "term_id": "GO:0006357",
  "gene": "UniProtKB:Q6VB84",
  "gene_symbol": "FOXD4L3",
  "gene_name": "Forkhead box protein D4-like 3"
}